oxalate catabolic process [GO:0033611] (biological process) Also known as: ethanedioate catabolic process, ethanedioic acid catabolic process, oxalate breakdown, oxalate catabolism, oxalate degradation, oxalic acid catabolic process Sources: GOC:mlg Definition: The chemical reactions and pathways resulting in the breakdown of oxalate, the organic acid ethanedioate. Relationships: is a type of oxalate metabolic process [GO:0033609]; is a type of GO:0043649